{
  "gene_symbol": "MAP7D2",
  "gene": "UniProtKB:Q96T17",
  "term_label": "microtubule cytoskeleton organization",
  "gene_name": "MAP7 domain-containing protein 2",
  "term_id": "GO:0000226"
}